{
  "term_id": "GO:0008063",
  "gene_name": "Interleukin-1 receptor-associated kinase 4",
  "gene_symbol": "IRAK4",
  "gene": "UniProtKB:Q9NWZ3",
  "term_label": "Toll signaling pathway"
}